phycoerythrobilin:ferredoxin oxidoreductase activity [GO:0050618] (MF) Definition: Catalysis of the reaction: (3Z)-phycoerythrobilin + oxidized ferredoxin = 15,16-dihydrobiliverdin + reduced ferredoxin. Relationships: is a type of oxidoreductase activity, acting on the CH-CH group of donors, iron-sulfur protein as acceptor [GO:0016636] Sources: EC:1.3.7.3, MetaCyc:1.3.7.3-RXN Also known as: (3Z)-phycoerythrobilin:ferredoxin oxidoreductase activity, PebB